regulation of tetrapyrrole catabolic process [GO:1901404] (biological process) Also known as: regulation of tetrapyrrole breakdown, regulation of tetrapyrrole catabolism, regulation of tetrapyrrole degradation Subtypes: GO:0010271, negative regulation of tetrapyrrole catabolic process [GO:1901405], GO:1901406 Relationships: is a type of regulation of catabolic process [GO:0009894]; is a type of regulation of tetrapyrrole metabolic process [GO:1901401]; RO_0002211 tetrapyrrole catabolic process [GO:0033015] Sources: GOC:TermGenie, GOC:mengo_curators Definition: Any process that modulates the frequency, rate or extent of tetrapyrrole catabolic process.